{
  "term_label": "regulation of transcription by RNA polymerase II",
  "gene_symbol": "HOXA5",
  "gene": "UniProtKB:P20719",
  "gene_name": "Homeobox protein Hox-A5",
  "term_id": "GO:0006357"
}